{
  "term_id": "GO:0030141",
  "term_label": "secretory granule",
  "gene": "UniProtKB:P49862",
  "gene_name": "Kallikrein-7",
  "gene_symbol": "KLK7"
}